{
  "term_id": "GO:0005737",
  "gene": "UniProtKB:P10398",
  "gene_name": "Serine_threonine-protein kinase A-Raf",
  "gene_symbol": "ARAF",
  "term_label": "cytoplasm"
}